{
  "term_id": "UNKNOWN:0001",
  "term_label": "Unknown molecular function",
  "gene_symbol": "WDR55",
  "gene": "UniProtKB:Q9H6Y2",
  "gene_name": "WD repeat-containing protein 55"
}